{
  "gene_name": "Transmembrane protein 17",
  "gene": "UniProtKB:Q86X19",
  "term_id": "GO:1905515",
  "gene_symbol": "TMEM17",
  "term_label": "non-motile cilium assembly"
}